{
  "term_id": "GO:0042102",
  "term_label": "positive regulation of T cell proliferation",
  "gene": "UniProtKB:P40933",
  "gene_name": "Interleukin-15",
  "gene_symbol": "IL15"
}